polarized epithelial cell differentiation [GO:0030859] (biological process) Definition: The process in which a relatively unspecialized cell acquires specialized features of a polarized epithelial cell. The polarized epithelial cell can be any of the cells within an epithelium where the epithelial sheet is oriented with respect to the planar axis. Subtypes: GO:0045198 Relationships: is a type of epithelial cell differentiation [GO:0030855]; is part of morphogenesis of a polarized epithelium [GO:0001738] Sources: GOC:mah Regulation: regulated by regulation of polarized epithelial cell differentiation [GO:0030860]; RO_0002212 by GO:0030861; positively regulated by positive regulation of polarized epithelial cell differentiation [GO:0030862]